{
  "gene_name": "Protocadherin gamma-A5",
  "gene_symbol": "PCDHGA5",
  "term_id": "GO:0050839",
  "gene": "UniProtKB:Q9Y5G8",
  "term_label": "cell adhesion molecule binding"
}